{
  "gene_symbol": "TCERG1L",
  "term_label": "nucleus",
  "gene_name": "Transcription elongation regulator 1-like protein",
  "term_id": "GO:0005634",
  "gene": "UniProtKB:Q5VWI1"
}